{
  "term_id": "UNKNOWN:0001",
  "gene": "UniProtKB:Q6NVV7",
  "gene_symbol": "CDPF1",
  "gene_name": "Cysteine-rich DPF motif domain-containing protein 1",
  "term_label": "Unknown molecular function"
}